negative regulation of CD4-positive, alpha-beta T cell differentiation [GO:0043371] (BP) Note: Note that immunologists typically use the word 'development' to refer to cells of B or T cell lineages undergoing the process that GO describes as 'cell differentiation'. Subtypes: negative regulation of CD4-positive, CD25-positive, alpha-beta regulatory T cell differentiation [GO:0032830], negative regulation of T-helper cell differentiation [GO:0045623] Relationships: is a type of regulation of CD4-positive, alpha-beta T cell differentiation [GO:0043370]; is a type of negative regulation of alpha-beta T cell differentiation [GO:0046639]; is a type of negative regulation of CD4-positive, alpha-beta T cell activation [GO:2000515]; negatively regulates CD4-positive, alpha-beta T cell differentiation [GO:0043367] Also known as: down regulation of CD4-positive, alpha beta T cell differentiation, down-regulation of CD4-positive, alpha beta T cell differentiation, downregulation of CD4-positive, alpha beta T cell differentiation, negative regulation of CD4-positive T-cell differentiation, negative regulation of CD4-positive T-lymphocyte differentiation, negative regulation of CD4-positive, alpha beta T lymphocyte differentiation, negative regulation of CD4-positive, alpha beta T-cell differentiation, negative regulation of CD4-positive, alpha beta T-lymphocyte differentiation, inhibition of CD4-positive, alpha beta T cell differentiation, negative regulation of CD4-positive, alpha beta T cell development Definition: Any process that stops, prevents, or reduces the frequency, rate, or extent of CD4-positive, alpha-beta T cell differentiation. Sources: GOC:add, GOC:pr, ISBN:0781735149